{
  "term_id": "GO:0006368",
  "gene_name": "Transcription elongation factor A protein 2",
  "gene": "UniProtKB:Q15560",
  "term_label": "transcription elongation by RNA polymerase II",
  "gene_symbol": "TCEA2"
}